DIM/DIP cell wall layer [GO:0097735] (cellular component) Definition: A section of the Actinobacterium-type cell wall composed of (phenyl)phthiocerol, phthiodiolone, phthiotriol dimycocerosate, diphthioceranate and other compounds. Sources: GOC:pr Relationships: is a type of GO:0110165; is part of Gram-positive-bacterium-type cell wall [GO:0009275]